{
  "gene_name": "Peripherin",
  "gene": "UniProtKB:P41219",
  "gene_symbol": "PRPH",
  "term_label": "intermediate filament organization",
  "term_id": "GO:0045109"
}